{
  "term_label": "sequence-specific DNA binding",
  "gene_symbol": "PGBD2",
  "gene": "UniProtKB:Q6P3X8",
  "term_id": "GO:0043565",
  "gene_name": "PiggyBac transposable element-derived protein 2"
}